{
  "term_label": "membrane",
  "term_id": "GO:0016020",
  "gene_name": "Transmembrane protein 91",
  "gene_symbol": "TMEM91",
  "gene": "UniProtKB:Q6ZNR0"
}